{
  "gene_symbol": "LPXN",
  "gene_name": "Leupaxin",
  "term_label": "negative regulation of B cell receptor signaling pathway",
  "gene": "UniProtKB:O60711",
  "term_id": "GO:0050859"
}